lateral root formation [GO:0010311] (biological process) Definition: The process that gives rise to a lateral root. This process pertains to the initial formation of a structure from unspecified parts. A lateral root primordium represents an organized group of cells derived from the root pericycle that will differentiate into a new root, as opposed to the initiation of the main root from the embryo proper. Relationships: is a type of GO:0009791; is a type of plant organ formation [GO:1905393]; BFO_0000050 lateral root morphogenesis [GO:0010102] Also known as: lateral root primordium development References: PMID:17259263 Sources: GOC:tair_curators